septin filament array [GO:0032160] (cellular component) Definition: Arrays of septin filaments, or bars, found in a series of filamentous structures. Such structures have been observed in the prospore membrane during spore formation in S. cerevisiae and in the chlamydospore membrane during chlamydospore formation in C. albicans. References: PMID:16151244 Sources: GOC:krc Also known as: septin bar Relationships: is a type of septin cytoskeleton [GO:0032156]; is part of GO:0005856 Subtypes: GO:0032165, chlamydospore septin filament array [GO:0032166]